regulation of imaginal disc-derived wing size [GO:0044719] (biological process) References: PMID:21393605 Definition: Any process that modulates the size of an imaginal disc-derived wing. Subtypes: GO:0044720, positive regulation of imaginal disc-derived wing size [GO:0120198] Relationships: is a type of regulation of anatomical structure size [GO:0090066]; is part of imaginal disc-derived wing morphogenesis [GO:0007476]